light transducer activity [GO:0031993] (molecular function) Definition: Absorbing energy from one or more photons and transferring their energy to another molecule, usually a protein, within the cell. Relationships: is a type of energy transducer activity [GO:0031992]; is part of GO:0009583 Sources: GOC:mah, GOC:mlg